{
  "gene": "UniProtKB:Q8TCN5",
  "gene_name": "Zinc finger protein 507",
  "term_label": "regulation of DNA-templated transcription",
  "gene_symbol": "ZNF507",
  "term_id": "GO:0006355"
}